SA node cell to atrial cardiac muscle cell communication by electrical coupling [GO:0086021] (biological process) Relationships: is a type of GO:0086064; is a type of GO:0086070 Also known as: SA node cardiac muscle cell to atrial cardiac muscle cell communication by electrical coupling, SA node cardiomyocyte to atrial cardiomyocyte communication by electrical coupling, SAN cardiomyocyte to atrial cardiomyocyte communication by electrical coupling, sinoatrial node cardiomyocyte to atrial cardiomyocyte communication by electrical coupling, sinus node cardiomyocyte to atrial cardiomyocyte communication by electrical coupling Sources: GOC:BHF, GOC:mtg_cardiac_conduct_nov11 Definition: The process that mediates signaling interactions between an SA node cardiomyocyte and an atrial cardiomyocyte by transfer of current between their adjacent cytoplasms via intercellular protein channels.